fucose biosynthetic process [GO:0042353] (BP) Definition: The chemical reactions and pathways resulting in the formation of fucose (6-deoxygalactose). Subtypes: L-fucose biosynthetic process [GO:0006005] Also known as: fucose anabolism, fucose biosynthesis, fucose formation, fucose synthesis Relationships: is a type of fucose metabolic process [GO:0006004]; is a type of hexose biosynthetic process [GO:0019319] Sources: GOC:jl